cardiac muscle cell action potential [GO:0086001] (biological process) Definition: An action potential that occurs in a cardiac muscle cell. Subtypes: cardiac muscle cell action potential involved in contraction [GO:0086002], GO:0086015, AV node cell action potential [GO:0086016], Purkinje myocyte action potential [GO:0086017], bundle of His cell action potential [GO:0086043] Regulation: RO_0002211 by stretch-activated, monoatomic cation-selective, calcium channel activity involved in regulation of cardiac muscle cell action potential [GO:0097365]; regulated by regulation of cardiac muscle cell action potential [GO:0098901] Sources: GOC:BHF, GOC:mtg_cardiac_conduct_nov11 Relationships: is a type of action potential [GO:0001508]